{
  "term_id": "GO:0048252",
  "gene_name": "Cytochrome P450 4A11",
  "gene_symbol": "CYP4A11",
  "term_label": "lauric acid metabolic process",
  "gene": "UniProtKB:Q02928"
}